palmitoyl-[glycerolipid] 3-(E)-desaturase activity [GO:0102654] (molecular function) Definition: Catalysis of the reaction: a 1-acyl-2-hexadecanoyl-glycerolipid + 2 H+ + O2 + 2 reduced [2Fe-2S]-[ferredoxin] = a 1-acyl-2-[(3E)-hexadec-3-enoyl]-glycerolipid + 2 H2O + 2 oxidized [2Fe-2S]-[ferredoxin]. The this activity introduces an unusual trans double bond at carbon 3 of a palmitoyl group attached to the sn-2 position of glycerolipids. Sources: RHEA:46764 Relationships: is a type of oxidoreductase activity, acting on paired donors, with oxidation of a pair of donors resulting in the reduction of molecular oxygen to two molecules of water [GO:0016717] Also known as: 1-18:1-2-16:0-phosphatidylglycerol trans-3 desaturase activity